{
  "term_label": "calcium ion binding",
  "gene_name": "Hippocalcin-like protein 1",
  "gene": "UniProtKB:P37235",
  "term_id": "GO:0005509",
  "gene_symbol": "HPCAL1"
}